{
  "gene_symbol": "SMIM11",
  "gene": "UniProtKB:P58511",
  "term_label": "Unknown biological process",
  "term_id": "UNKNOWN:0002",
  "gene_name": "Small integral membrane protein 11"
}